{
  "gene_symbol": "FAM133B",
  "gene": "UniProtKB:Q5BKY9",
  "term_label": "Unknown biological process",
  "term_id": "UNKNOWN:0002",
  "gene_name": "Protein FAM133B"
}